{
  "gene": "UniProtKB:Q8TE96",
  "term_label": "spliceosomal complex",
  "term_id": "GO:0005681",
  "gene_symbol": "DQX1",
  "gene_name": "ATP-dependent RNA helicase DQX1"
}